{
  "gene": "UniProtKB:Q9UKT7",
  "gene_name": "F-box_LRR-repeat protein 3",
  "term_label": "cytosol",
  "gene_symbol": "FBXL3",
  "term_id": "GO:0005829"
}